{
  "term_label": "Unknown biological process",
  "gene_symbol": "IAPP",
  "gene_name": "Islet amyloid polypeptide",
  "term_id": "UNKNOWN:0002",
  "gene": "UniProtKB:P10997"
}